{
  "term_id": "GO:0048813",
  "gene_symbol": "ABITRAM",
  "gene_name": "Protein Abitram",
  "term_label": "dendrite morphogenesis",
  "gene": "UniProtKB:Q9NX38"
}